{
  "term_label": "Unknown molecular function",
  "gene": "UniProtKB:Q3KNT9",
  "gene_symbol": "TMEM95",
  "gene_name": "Sperm-egg fusion protein TMEM95",
  "term_id": "UNKNOWN:0001"
}